{
  "gene": "UniProtKB:Q9HCS7",
  "gene_symbol": "XAB2",
  "term_label": "U2-type catalytic step 2 spliceosome",
  "gene_name": "Pre-mRNA-splicing factor SYF1",
  "term_id": "GO:0071007"
}